fonsecin catabolic process [GO:1900768] (biological process) Definition: The chemical reactions and pathways resulting in the breakdown of fonsecin. Sources: GOC:TermGenie, GOC:di Also known as: fonsecin breakdown, fonsecin catabolism, fonsecin degradation Relationships: is a type of GO:0019336; is a type of polyketide catabolic process [GO:0030640]; is a type of alcohol catabolic process [GO:0046164]; is a type of naphtho-gamma-pyrone catabolic process [GO:1900786]; is a type of ether catabolic process [GO:1901502]